dormancy process [GO:0022611] (biological process) Subtypes: seed dormancy process [GO:0010162], GO:0042750, estivation [GO:0042751], entry into diapause [GO:0055115], exit from diapause [GO:0071981], maintenance of diapause [GO:0071982], GO:0075214, GO:0085014, dormancy maintenance of symbiont in host [GO:0085015], dormancy exit of symbiont in host [GO:0085016], GO:0097207, entry into dormancy [GO:0097436], maintenance of dormancy [GO:0097437], exit from dormancy [GO:0097438], GO:0097439 Also known as: multicellular organism dormancy process, spore dormancy process Sources: GOC:PO_curators, GOC:isa_complete, PO_REF:00009 Note: In plants and animals, dormancy may be a response to environmental conditions such as seasonality or extreme heat, drought, or cold. In plants, dormancy may involve the formation of dormant buds, and may be preceded by the senescence of plant parts such as leaves in woody plants or most of the shoot system in herbaceous perennials. The exit from dormancy in vascular plants is marked by resumed growth of buds and/or growth of vascular cambium. Definition: A developmental process in which dormancy (sometimes called a dormant state) is induced, maintained or broken. Dormancy is a suspension of most physiological activity and growth that can be reactivated. Relationships: is_a developmental process [GO:0032502]